{
  "term_id": "GO:0031012",
  "gene_name": "Galectin-3",
  "gene_symbol": "LGALS3",
  "gene": "UniProtKB:P17931",
  "term_label": "extracellular matrix"
}